5-oxovalerate dehydrogenase activity [GO:0055043] (molecular function) Definition: Catalysis of the reaction: 5-oxovalerate + NADP+ + H2O = glutarate + NADPH + H+. Sources: GOC:jid, GOC:mlg Relationships: is a type of oxidoreductase activity, acting on the aldehyde or oxo group of donors, NAD or NADP as acceptor [GO:0016620]